2,4-dichlorophenol 6-monooxygenase activity [GO:0018666] (molecular function) Definition: Catalysis of the reaction: 2,4-dichlorophenol + NADPH + H+ + O2 = 3,5-dichlorocatechol + NADP+ + H2O. Sources: EC:1.14.13.20 Also known as: 2,4-dichlorophenol hydroxylase activity, 2,4-dichlorophenol monooxygenase activity, 2,4-dichlorophenol,NADPH:oxygen oxidoreductase (6-hydroxylating) Relationships: is a type of oxidoreductase activity, acting on paired donors, with incorporation or reduction of molecular oxygen, NAD(P)H as one donor, and incorporation of one atom of oxygen [GO:0016709]